octopamine secretion [GO:0061539] (biological process) Definition: The controlled release of octopamine by a cell. Sources: GOC:dph Subtypes: octopamine secretion, neurotransmission [GO:0061540] Relationships: is a type of organic cation transport [GO:0015695]; is a type of GO:0015850; is a type of secretion by cell [GO:0032940]; is a type of nitrogen compound transport [GO:0071705]